orlandin biosynthetic process [GO:1900821] (biological process) Sources: GOC:TermGenie, GOC:di Relationships: is a type of secondary metabolite biosynthetic process [GO:0044550]; is_a GO:1900819 Definition: The chemical reactions and pathways resulting in the formation of orlandin. Also known as: orlandin anabolism, orlandin biosynthesis, orlandin formation, orlandin synthesis